{
  "gene_symbol": "HKDC1",
  "gene_name": "Hexokinase HKDC1",
  "term_label": "fructokinase activity",
  "gene": "UniProtKB:Q2TB90",
  "term_id": "GO:0008865"
}